25-hydroxycholecalciferol-24-hydroxylase activity [GO:0008403] (MF) Definition: Catalysis of the hydroxylation of C-24 of 25-hydroxycholecalciferol (25-hydroxyvitamin D3) to form 24(R),25-dihydroxycholecalciferol. Relationships: is a type of GO:0016705; is a type of GO:0070576 Sources: ISBN:0471331309 Also known as: 25-hydroxyvitamin D3 24-hydroxylase activity, cytochrome P450 CYP24